intermediate-density lipoprotein particle binding [GO:0071815] (molecular function) Relationships: is a type of GO:0071813 Also known as: IDL binding, intermediate-density lipoprotein binding Sources: GOC:BHF, GOC:mah Definition: Binding to a intermediate-density lipoprotein particle, a triglyceride-rich lipoprotein particle that typically contains APOB100, APOE and APOCs and has a density of 1.006-1.019 g/ml and a diameter of between 25-30 nm.